{
  "term_id": "GO:0019901",
  "gene": "UniProtKB:Q9Y2T1",
  "gene_symbol": "AXIN2",
  "gene_name": "Axin-2",
  "term_label": "protein kinase binding"
}